{
  "term_id": "GO:0000226",
  "term_label": "microtubule cytoskeleton organization",
  "gene_symbol": "CETN3",
  "gene_name": "Centrin-3",
  "gene": "UniProtKB:O15182"
}